regulation of T cell tolerance induction to tumor cell [GO:0002846] (biological process) Subtypes: negative regulation of T cell tolerance induction to tumor cell [GO:0002847], positive regulation of T cell tolerance induction to tumor cell [GO:0002848] Relationships: is a type of GO:0002840; is a type of regulation of tolerance induction to tumor cell [GO:0002843]; is_a GO:0002849; regulates T cell tolerance induction to tumor cell [GO:0002411] Sources: GOC:add Definition: Any process that modulates the frequency, rate, or extent of T cell tolerance induction to tumor cell.